{
  "gene_symbol": "A0A8Q3WLD3",
  "term_id": "UNKNOWN:0001",
  "gene_name": "Uncharacterized protein",
  "gene": "UniProtKB:A0A8Q3WLD3",
  "term_label": "Unknown molecular function"
}